vocal learning [GO:0042297] (biological process) Relationships: is a type of auditory behavior [GO:0031223]; is a type of imitative learning [GO:0098596]; is a type of learned vocalization behavior or vocal learning [GO:0098598] References: PMID:16418265, PMID:17035521 Sources: GOC:BHF, GOC:dos, GOC:rl Note: Examples include language learning by human infants and song learning in zebra finches. Definition: A behavioral process whose outcome is a relatively long-lasting behavioral change whereby an organism modifies innate vocalizations to imitate sounds produced by others.